{
  "gene": "UniProtKB:Q9H756",
  "gene_symbol": "LRRC19",
  "term_label": "signaling receptor activity",
  "term_id": "GO:0038023",
  "gene_name": "Leucine-rich repeat-containing protein 19"
}